{
  "gene_name": "Formin-like protein 2",
  "gene": "UniProtKB:Q96PY5",
  "term_label": "cortical actin cytoskeleton organization",
  "gene_symbol": "FMNL2",
  "term_id": "GO:0030866"
}